positive regulation of hypersensitivity [GO:0002885] (biological process) Definition: Any process that activates or increases the frequency, rate, or extent of hypersensitivity. Relationships: is a type of positive regulation of acute inflammatory response to antigenic stimulus [GO:0002866]; is_a regulation of hypersensitivity [GO:0002883]; positively regulates hypersensitivity [GO:0002524] Sources: GOC:add Also known as: up regulation of hypersensitivity, up-regulation of hypersensitivity, upregulation of hypersensitivity, activation of hypersensitivity, stimulation of hypersensitivity Subtypes: positive regulation of type III hypersensitivity [GO:0001805], positive regulation of type IV hypersensitivity [GO:0001809], positive regulation of type I hypersensitivity [GO:0001812], positive regulation of type II hypersensitivity [GO:0002894]